{
  "term_id": "GO:0031122",
  "gene_name": "Cytoplasmic dynein 1 heavy chain 1",
  "gene": "UniProtKB:Q14204",
  "term_label": "cytoplasmic microtubule organization",
  "gene_symbol": "DYNC1H1"
}